{
  "gene": "UniProtKB:Q14642",
  "gene_name": "Inositol polyphosphate-5-phosphatase A",
  "gene_symbol": "INPP5A",
  "term_label": "inositol-polyphosphate 5-phosphatase activity",
  "term_id": "GO:0004445"
}